negative regulation of motile cilium assembly [GO:1905504] (biological process) Also known as: inhibition of motile primary cilia assembly, inhibition of motile primary cilia formation, inhibition of motile primary cilium assembly, inhibition of motile primary cilium formation, down regulation of motile primary cilia assembly, down regulation of motile primary cilia formation, down regulation of motile primary cilium assembly, down regulation of motile primary cilium formation, down regulation of nodal cilium assembly, down regulation of nodal cilium formation, down-regulation of motile primary cilia assembly, down-regulation of motile primary cilia formation, down-regulation of motile primary cilium assembly, down-regulation of motile primary cilium formation, down-regulation of nodal cilium assembly, down-regulation of nodal cilium formation, downregulation of motile primary cilia assembly, downregulation of motile primary cilia formation, downregulation of motile primary cilium assembly, downregulation of motile primary cilium formation, downregulation of nodal cilium assembly, downregulation of nodal cilium formation, inhibition of nodal cilium assembly, inhibition of nodal cilium formation, negative regulation of motile primary cilia assembly, negative regulation of motile primary cilia formation, negative regulation of motile primary cilium assembly, negative regulation of motile primary cilium formation, negative regulation of nodal cilium assembly, negative regulation of nodal cilium formation Definition: Any process that stops, prevents or reduces the frequency, rate or extent of motile cilium assembly. References: PMID:25294941 Sources: GOC:TermGenie, GOC:cilia, GOC:krc, GO_REF:0000058 Relationships: is a type of GO:1902018; is a type of regulation of motile cilium assembly [GO:1905503]; RO_0002212 GO:0044458